{
  "term_label": "glycerol biosynthetic process from pyruvate",
  "term_id": "GO:0046327",
  "gene_symbol": "PCK2",
  "gene": "UniProtKB:Q16822",
  "gene_name": "Phosphoenolpyruvate carboxykinase [GTP], mitochondrial"
}